{
  "term_label": "Unknown cellular component",
  "term_id": "UNKNOWN:0003",
  "gene": "UniProtKB:Q99590",
  "gene_name": "Protein SCAF11",
  "gene_symbol": "SCAF11"
}